mammary gland epithelial cell differentiation [GO:0060644] (BP) Definition: The process in which a relatively unspecialized epithelial cell becomes a more specialized epithelial cell of the mammary gland. Sources: GOC:dph Relationships: is_a GO:0030855; is part of GO:0061180 Subtypes: epithelial cell differentiation involved in mammary gland bud morphogenesis [GO:0060643], GO:0060653, epithelial cell differentiation involved in mammary gland alveolus development [GO:0061030]